{
  "gene_name": "Olfactory receptor 6C1",
  "gene": "UniProtKB:Q96RD1",
  "term_id": "GO:0004984",
  "term_label": "olfactory receptor activity",
  "gene_symbol": "OR6C1"
}